{
  "term_label": "diadenosine tetraphosphate biosynthetic process",
  "gene_name": "Lysine--tRNA ligase",
  "gene_symbol": "KARS1",
  "term_id": "GO:0015966",
  "gene": "UniProtKB:Q15046"
}